{
  "gene": "UniProtKB:Q9C0A0",
  "term_id": "GO:0007399",
  "term_label": "nervous system development",
  "gene_name": "Contactin-associated protein-like 4",
  "gene_symbol": "CNTNAP4"
}